trans-Golgi network membrane organization [GO:0098629] (biological process) Relationships: is a type of membrane organization [GO:0061024] Definition: A process which results in the assembly, arrangement of constituent parts, or disassembly of a trans-Golgi network membrane. References: PMID:23345439 Sources: GOC:di, GOC:dos